{
  "term_label": "flavin adenine dinucleotide binding",
  "gene_symbol": "GCDH",
  "gene": "UniProtKB:Q92947",
  "term_id": "GO:0050660",
  "gene_name": "Glutaryl-CoA dehydrogenase, mitochondrial"
}